{
  "gene": "UniProtKB:Q8NH53",
  "term_label": "plasma membrane",
  "gene_name": "Olfactory receptor 52N1",
  "gene_symbol": "OR52N1",
  "term_id": "GO:0005886"
}